{
  "gene_name": "CKLF-like MARVEL transmembrane domain-containing protein 3",
  "term_id": "UNKNOWN:0002",
  "gene": "UniProtKB:Q96MX0",
  "term_label": "Unknown biological process",
  "gene_symbol": "CMTM3"
}